{
  "term_id": "GO:0004585",
  "gene": "UniProtKB:P00480",
  "gene_symbol": "OTC",
  "gene_name": "Ornithine transcarbamylase, mitochondrial",
  "term_label": "ornithine carbamoyltransferase activity"
}